negative regulation of spontaneous neurotransmitter secretion [GO:1904049] (biological process) Definition: Any process that stops, prevents or reduces the frequency, rate or extent of spontaneous neurotransmitter secretion. Also known as: down regulation of spontaneous neurotransmitter secretion, down regulation of stimulus-independent neurotransmitter secretion, down-regulation of spontaneous neurotransmitter secretion, down-regulation of stimulus-independent neurotransmitter secretion, downregulation of spontaneous neurotransmitter secretion, downregulation of stimulus-independent neurotransmitter secretion, negative regulation of stimulus-independent neurotransmitter secretion, inhibition of spontaneous neurotransmitter secretion, inhibition of stimulus-independent neurotransmitter secretion References: PMID:22314364 Sources: GOC:PARL, GOC:TermGenie, GOC:pad, GO_REF:0000058 Relationships: is a type of GO:0046929; is a type of regulation of spontaneous neurotransmitter secretion [GO:1904048]; negatively regulates spontaneous neurotransmitter secretion [GO:0061669] Note: An example of this is PARK2 / parkin in human (O60260) in PMID:22314364 (inferred from mutant phenotype).